{
  "gene_name": "Olfactory receptor 4S1",
  "term_id": "UNKNOWN:0002",
  "gene": "UniProtKB:Q8NGB4",
  "gene_symbol": "OR4S1",
  "term_label": "Unknown biological process"
}